{
  "gene_name": "Protein phosphatase Slingshot homolog 1",
  "term_label": "cytoplasm",
  "gene": "UniProtKB:Q8WYL5",
  "term_id": "GO:0005737",
  "gene_symbol": "SSH1"
}